{
  "gene": "UniProtKB:Q8WWX8",
  "term_label": "myo-inositol transmembrane transporter activity",
  "term_id": "GO:0005365",
  "gene_symbol": "SLC5A11",
  "gene_name": "Sodium_myo-inositol cotransporter 2"
}